error-free translesion synthesis [GO:0070987] (biological process) Relationships: is a type of translesion synthesis [GO:0019985] Sources: GOC:elh Note: Note that 'error-free' does not mean that literally zero errors occur during DNA synthesis, but that the error rate is low, comparable to that of DNA synthesis during replication. Definition: The conversion of DNA-damage induced single-stranded gaps into large molecular weight DNA after replication by using a specialized DNA polymerase or replication complex to insert a defined nucleotide across the lesion. This process does not remove the replication-blocking lesions but does not causes an increase in the endogenous mutation level. For S. cerevisiae, RAD30 encodes DNA polymerase eta, which incorporates two adenines. When incorporated across a thymine-thymine dimer, it does not increase the endogenous mutation level.